positive regulation of cell budding [GO:0045782] (biological process) Relationships: is a type of GO:0007116; is a type of GO:0051781; is a type of positive regulation of asexual reproduction [GO:1903666]; positively regulates GO:0007114 Definition: Any process that activates or increases the frequency, rate or extent of cell budding. Also known as: positive regulation of budding, up regulation of cell budding, up-regulation of cell budding, upregulation of cell budding, activation of cell budding, stimulation of cell budding Sources: GOC:go_curators